MHC class Ib protein binding, via lateral surface [GO:0023031] (molecular function) Definition: Binding to a major histocompatibility complex class Ib molecules via the lateral surface. Sources: GOC:mtg_signal, GOC:vw Relationships: is a type of MHC class Ib protein binding [GO:0023029]